{
  "term_id": "GO:0042981",
  "term_label": "regulation of apoptotic process",
  "gene": "UniProtKB:Q13075",
  "gene_symbol": "NAIP",
  "gene_name": "Baculoviral IAP repeat-containing protein 1"
}